positive regulation of natural killer cell proliferation involved in immune response [GO:0032822] (BP) Relationships: is_a positive regulation of immune effector process [GO:0002699]; is a type of positive regulation of natural killer cell proliferation [GO:0032819]; is a type of regulation of natural killer cell proliferation involved in immune response [GO:0032820]; positively regulates natural killer cell proliferation involved in immune response [GO:0002324] Definition: Any process that activates or increases the frequency, rate or extent of natural killer cell proliferation as part of an immune response. Sources: GOC:mah Also known as: activation of natural killer cell proliferation during immune response, stimulation of natural killer cell proliferation during immune response, positive regulation of NK cell proliferation during immune response, positive regulation of natural killer cell proliferation during immune response, up regulation of natural killer cell proliferation during immune response, up-regulation of natural killer cell proliferation during immune response, upregulation of natural killer cell proliferation during immune response